negative regulation of mitotic spindle formation (spindle phase one) [GO:0110160] (biological process) Definition: Any process that stops, prevents or reduces the frequency, rate or extent of the cell cycle process in which the distance is lengthened between poles of the mitotic spindle during mitotic prophase (spindle phase one). Sources: GOC:vw Relationships: is a type of regulation of mitotic spindle formation (spindle phase one) [GO:0110159]; is a type of negative regulation of spindle assembly [GO:1905831]; negatively regulates mitotic spindle formation (spindle phase one) [GO:0061804]